{
  "gene_name": "Protein Abitram",
  "gene": "UniProtKB:Q9NX38",
  "gene_symbol": "ABITRAM",
  "term_label": "regulation of actin filament polymerization",
  "term_id": "GO:0030833"
}